{
  "term_id": "UNKNOWN:0002",
  "term_label": "Unknown biological process",
  "gene": "UniProtKB:A6NDX4",
  "gene_symbol": "A6NDX4",
  "gene_name": "Putative transmembrane protein ENSP00000320207"
}